{
  "term_id": "UNKNOWN:0001",
  "gene_symbol": "TRAV38-1",
  "gene": "UniProtKB:A0A0B4J264",
  "gene_name": "T cell receptor alpha variable 38-1",
  "term_label": "Unknown molecular function"
}